{
  "term_label": "estrogen metabolic process",
  "term_id": "GO:0008210",
  "gene_symbol": "CYP1B1",
  "gene": "UniProtKB:Q16678",
  "gene_name": "Cytochrome P450 1B1"
}